{
  "gene_symbol": "NOMO2",
  "term_label": "endoplasmic reticulum membrane",
  "gene_name": "BOS complex subunit NOMO2",
  "gene": "UniProtKB:Q5JPE7",
  "term_id": "GO:0005789"
}